viral membrane [GO:0036338] (cellular component) Definition: The lipid bilayer of a virion, a complete fully infectious extracellular virus particle. Relationships: is_a virion component [GO:0044423] Subtypes: viral envelope [GO:0019031], GO:0039641 Sources: GOC:bm